{
  "term_label": "inhibitory synapse assembly",
  "gene": "UniProtKB:P78334",
  "gene_symbol": "GABRE",
  "gene_name": "Gamma-aminobutyric acid receptor subunit epsilon",
  "term_id": "GO:1904862"
}